N-terminal protein amino acid deamination, from side chain [GO:0031364] (biological process) Sources: GOC:mah Relationships: is a type of N-terminal protein amino acid deamination [GO:0031363] Definition: The removal of an amino group from the side chain of an N-terminal asparagine or glutamine residue of a protein.